{
  "term_label": "ATP citrate synthase activity",
  "term_id": "GO:0003878",
  "gene_symbol": "ACLY",
  "gene": "UniProtKB:P53396",
  "gene_name": "ATP-citrate synthase"
}